{
  "gene_symbol": "KCNA1",
  "term_id": "GO:0016020",
  "term_label": "membrane",
  "gene": "UniProtKB:Q09470",
  "gene_name": "Potassium voltage-gated channel subfamily A member 1"
}